negative regulation of double-strand break repair via single-strand annealing [GO:1901291] (biological process) Also known as: down regulation of double-strand break repair via single-strand annealing, down-regulation of double-strand break repair via single-strand annealing, downregulation of double-strand break repair via single-strand annealing, inhibition of double-strand break repair via single-strand annealing Sources: GOC:TermGenie, GOC:sart Relationships: is a type of negative regulation of double-strand break repair [GO:2000780]; negatively regulates double-strand break repair via single-strand annealing [GO:0045002] Definition: Any process that stops, prevents or reduces the frequency, rate or extent of double-strand break repair via single-strand annealing.